{
  "term_label": "negative regulation of T cell proliferation",
  "gene": "UniProtKB:Q9NZQ7",
  "gene_name": "Programmed cell death 1 ligand 1",
  "gene_symbol": "CD274",
  "term_id": "GO:0042130"
}